{
  "gene_symbol": "KIF1C",
  "gene_name": "Kinesin-like protein KIF1C",
  "term_id": "GO:0005874",
  "gene": "UniProtKB:O43896",
  "term_label": "microtubule"
}